{
  "gene_name": "Insulin-induced gene 1 protein",
  "gene_symbol": "INSIG1",
  "gene": "UniProtKB:O15503",
  "term_label": "endoplasmic reticulum",
  "term_id": "GO:0005783"
}